{
  "gene_symbol": "EIF4EBP2",
  "gene_name": "Eukaryotic translation initiation factor 4E-binding protein 2",
  "term_label": "negative regulation of translational initiation",
  "gene": "UniProtKB:Q13542",
  "term_id": "GO:0045947"
}